{
  "term_label": "vocalization behavior",
  "term_id": "GO:0071625",
  "gene_name": "Forkhead box protein P2",
  "gene": "UniProtKB:O15409",
  "gene_symbol": "FOXP2"
}